L-histidine transport [GO:1902024] (biological process) Relationships: is a type of organic cation transport [GO:0015695]; is a type of aromatic amino acid transport [GO:0015801]; is a type of basic amino acid transport [GO:0015802]; is a type of GO:0015807 Subtypes: L-histidine transmembrane export from vacuole [GO:0089708], L-histidine transmembrane import into vacuole [GO:0090513] References: PMID:22822152 Sources: GOC:TermGenie, GOC:kmv Definition: The directed movement of a L-histidine into, out of or within a cell, or between cells, by means of some agent such as a transporter or pore.